{
  "term_id": "GO:0005615",
  "term_label": "extracellular space",
  "gene": "UniProtKB:Q2TAL6",
  "gene_name": "Brorin",
  "gene_symbol": "VWC2"
}